{
  "gene_symbol": "MAP1B",
  "term_label": "microtubule",
  "term_id": "GO:0005874",
  "gene": "UniProtKB:P46821",
  "gene_name": "Microtubule-associated protein 1B"
}